{
  "term_id": "UNKNOWN:0001",
  "term_label": "Unknown molecular function",
  "gene_symbol": "TRBV7-8",
  "gene_name": "T cell receptor beta variable 7-8",
  "gene": "UniProtKB:A0A1B0GX51"
}